{
  "gene_symbol": "GOLGB1",
  "gene": "UniProtKB:Q14789",
  "gene_name": "Golgin subfamily B member 1",
  "term_label": "cis-Golgi network",
  "term_id": "GO:0005801"
}